chemokine (C-C motif) ligand 21 signaling pathway [GO:0038116] (biological process) Also known as: CCL21-mediated signaling pathway, chemokine (C-C motif) ligand 21 signalling pathway, C-C chemokine receptor type 7 signaling pathway Note: The C-C chemokine CCL21 s a known agonist of the chemokine receptor type 7 (CCR7). Consider instead annotating to the child term 'CCL21-activated CCR7 signaling pathway ; GO:0038120'. Subtypes: GO:0038120 Relationships: is a type of GO:0070098 Definition: The series of molecular signals initiated by the binding of the C-C chemokine CCL21 to its receptor on the surface of a target cell, and ending with the regulation of a downstream cellular process, e.g. transcription. References: PMID:15059845 Sources: GOC:nhn, GOC:signaling